{
  "term_id": "GO:0008528",
  "term_label": "G protein-coupled peptide receptor activity",
  "gene_name": "Thyrotropin receptor",
  "gene_symbol": "TSHR",
  "gene": "UniProtKB:P16473"
}